{
  "gene_name": "CASP8-associated protein 2",
  "gene_symbol": "CASP8AP2",
  "term_label": "transcription corepressor activity",
  "gene": "UniProtKB:Q9UKL3",
  "term_id": "GO:0003714"
}